{
  "gene_symbol": "CPT1A",
  "term_label": "carnitine O-palmitoyltransferase activity",
  "gene": "UniProtKB:P50416",
  "term_id": "GO:0004095",
  "gene_name": "Carnitine O-palmitoyltransferase 1, liver isoform"
}